{
  "gene": "UniProtKB:Q5VVQ6",
  "gene_symbol": "YOD1",
  "term_label": "cysteine-type deubiquitinase activity",
  "gene_name": "Ubiquitin thioesterase OTU1",
  "term_id": "GO:0004843"
}